{
  "gene_symbol": "PPP1CC",
  "gene": "UniProtKB:P36873",
  "gene_name": "Serine_threonine-protein phosphatase PP1-gamma catalytic subunit",
  "term_id": "GO:0005737",
  "term_label": "cytoplasm"
}